{
  "term_label": "Unknown cellular component",
  "gene_name": "Immunoglobulin heavy variable 3-64D",
  "gene": "UniProtKB:A0A0J9YX35",
  "term_id": "UNKNOWN:0003",
  "gene_symbol": "IGHV3-64D"
}